{
  "gene_name": "Zinc finger protein 461",
  "gene_symbol": "ZNF461",
  "term_id": "GO:0000978",
  "gene": "UniProtKB:Q8TAF7",
  "term_label": "RNA polymerase II cis-regulatory region sequence-specific DNA binding"
}